{
  "gene": "UniProtKB:P18848",
  "term_id": "GO:1990590",
  "term_label": "ATF1-ATF4 transcription factor complex",
  "gene_symbol": "ATF4",
  "gene_name": "Cyclic AMP-dependent transcription factor ATF-4"
}